{
  "gene_name": "T cell receptor alpha joining 26 (Fragment)",
  "term_id": "UNKNOWN:0001",
  "gene_symbol": "TRAJ26",
  "term_label": "Unknown molecular function",
  "gene": "UniProtKB:A0A075B6V7"
}